positive regulation of [4Fe-4S] cluster assembly [GO:1900493] (biological process) Relationships: is a type of regulation of [4Fe-4S] cluster assembly [GO:1900491]; is a type of positive regulation of iron-sulfur cluster assembly [GO:1903331]; positively regulates [4Fe-4S] cluster assembly [GO:0044572] Sources: GOC:TermGenie, GOC:mengo_curators, GOC:pr Definition: Any process that activates or increases the frequency, rate or extent of [4Fe-4S] cluster assembly. Also known as: positive regulation of 4Fe-4S cluster assembly, up regulation of 4Fe-4S cluster assembly, up regulation of [4Fe-4S] cluster assembly, up-regulation of 4Fe-4S cluster assembly, up-regulation of [4Fe-4S] cluster assembly, upregulation of 4Fe-4S cluster assembly, upregulation of [4Fe-4S] cluster assembly, activation of 4Fe-4S cluster assembly, activation of [4Fe-4S] cluster assembly, activation of [4Fe-4S] cluster biosynthetic process, positive regulation of [4Fe-4S] cluster biosynthetic process, up regulation of [4Fe-4S] cluster biosynthetic process, up-regulation of [4Fe-4S] cluster biosynthetic process, upregulation of [4Fe-4S] cluster biosynthetic process